{
  "term_id": "GO:0061631",
  "gene": "UniProtKB:P62253",
  "term_label": "ubiquitin conjugating enzyme activity",
  "gene_name": "Ubiquitin-conjugating enzyme E2 G1",
  "gene_symbol": "UBE2G1"
}